sorocarp stalk morphogenesis [GO:0036360] (BP) Also known as: fruiting body stalk morphogenesis Relationships: is a type of anatomical structure morphogenesis [GO:0009653]; is part of GO:0031150; is part of sorocarp morphogenesis [GO:0031288] References: PMID:22902739 Sources: DDANAT:0000068, GOC:pf Definition: The process in which the sorocarp stalk is generated and organized. The sorocarp stalk is a tubular structure that consists of cellulose-covered cells stacked on top of each other and surrounded by an acellular stalk tube composed of cellulose and glycoprotein. An example of this process is found in Dictyostelium discoideum.